RNA cap binding complex [GO:0034518] (cellular component) Definition: A protein complex that binds to an RNA cap structure to mediate RNA processing and/or translation initiation. Relationships: is a type of intracellular protein-containing complex [GO:0140535] Sources: GOC:mah Subtypes: nuclear cap binding complex [GO:0005846], eukaryotic translation initiation factor 4F complex [GO:0016281]